{
  "gene_symbol": "REPS1",
  "term_id": "GO:0005737",
  "gene_name": "RalBP1-associated Eps domain-containing protein 1",
  "term_label": "cytoplasm",
  "gene": "UniProtKB:Q96D71"
}